{
  "term_label": "Unknown cellular component",
  "gene": "UniProtKB:Q9BVH7",
  "gene_symbol": "ST6GALNAC5",
  "gene_name": "Alpha-N-acetylgalactosaminide alpha-2,6-sialyltransferase 5",
  "term_id": "UNKNOWN:0003"
}